{
  "term_id": "GO:0005085",
  "gene": "UniProtKB:Q8TEU7",
  "gene_symbol": "RAPGEF6",
  "term_label": "guanyl-nucleotide exchange factor activity",
  "gene_name": "Rap guanine nucleotide exchange factor 6"
}